interleukin-12 alpha subunit binding [GO:0042164] (molecular function) Also known as: CLMFp35 binding, IL-12A binding, IL-12p35 binding, NKSFp35 binding Sources: GOC:mah Relationships: is a type of interleukin-12 binding [GO:0019972] Definition: Binding to the alpha subunit of interleukin-12.